{
  "gene": "UniProtKB:Q8N7H1",
  "gene_name": "Putative uncharacterized protein encoded by LINC01465",
  "gene_symbol": "LINC01465",
  "term_id": "UNKNOWN:0001",
  "term_label": "Unknown molecular function"
}